{
  "gene_symbol": "NBL1",
  "term_label": "receptor ligand activity",
  "gene_name": "Neuroblastoma suppressor of tumorigenicity 1",
  "gene": "UniProtKB:P41271",
  "term_id": "GO:0048018"
}